regulation of selenocysteine incorporation [GO:1904569] (biological process) Relationships: is_a regulation of translational elongation [GO:0006448]; regulates selenocysteine incorporation [GO:0001514] References: PMID:21685449 Sources: GOC:TermGenie, GO_REF:0000058 Subtypes: negative regulation of selenocysteine incorporation [GO:1904570], positive regulation of selenocysteine incorporation [GO:1904571] Definition: Any process that modulates the frequency, rate or extent of selenocysteine incorporation.